{
  "term_label": "heparan sulfate 6-sulfotransferase activity",
  "gene_name": "Heparan-sulfate 6-O-sulfotransferase 3",
  "gene_symbol": "HS6ST3",
  "gene": "UniProtKB:Q8IZP7",
  "term_id": "GO:0017095"
}